{
  "gene_name": "26S proteasome non-ATPase regulatory subunit 12",
  "gene_symbol": "PSMD12",
  "term_id": "GO:0005737",
  "term_label": "cytoplasm",
  "gene": "UniProtKB:O00232"
}